{
  "gene_symbol": "MGP",
  "gene_name": "Matrix Gla protein",
  "term_label": "Unknown molecular function",
  "term_id": "UNKNOWN:0001",
  "gene": "UniProtKB:P08493"
}